desmosome assembly [GO:0002159] (biological process) Sources: GOC:hjd, ISBN:0198506732 Relationships: is a type of desmosome organization [GO:0002934]; is a type of GO:0007043 Note: Desmosomes link two cells together; hemidesmosomes attach one cell to the extracellular matrix. Definition: A cellular process that results in the aggregation, arrangement and bonding together of a set of components to form a desmosome. A desmosome is a patch-like intercellular junction found in vertebrate tissues, consisting of parallel zones of two cell membranes, separated by an space of 25-35 nm, and having dense fibrillar plaques in the subjacent cytoplasm.